{
  "gene": "UniProtKB:P56715",
  "gene_symbol": "RP1",
  "gene_name": "Oxygen-regulated protein 1",
  "term_id": "GO:0060041",
  "term_label": "retina development in camera-type eye"
}